{
  "gene_symbol": "MMP12",
  "gene": "UniProtKB:P39900",
  "gene_name": "Macrophage metalloelastase",
  "term_label": "metalloendopeptidase activity",
  "term_id": "GO:0004222"
}